{
  "gene_name": "Sialate O-acetylesterase",
  "gene": "UniProtKB:Q9HAT2",
  "term_id": "GO:0001681",
  "gene_symbol": "SIAE",
  "term_label": "sialate O-acetylesterase activity"
}